{
  "gene_symbol": "AP5S1",
  "gene_name": "AP-5 complex subunit sigma-1",
  "term_id": "GO:0016197",
  "term_label": "endosomal transport",
  "gene": "UniProtKB:Q9NUS5"
}